{
  "term_id": "UNKNOWN:0001",
  "gene_symbol": "POLR3A",
  "gene_name": "DNA-directed RNA polymerase III subunit RPC1",
  "term_label": "Unknown molecular function",
  "gene": "UniProtKB:O14802"
}